{
  "gene_name": "Probable ubiquitin carboxyl-terminal hydrolase MINDY-4",
  "gene_symbol": "MINDY4",
  "gene": "UniProtKB:Q4G0A6",
  "term_id": "GO:1990380",
  "term_label": "K48-linked deubiquitinase activity"
}